{
  "term_label": "ubiquitin recycling",
  "gene_name": "Phospholipase A-2-activating protein",
  "term_id": "GO:0010992",
  "gene": "UniProtKB:Q9Y263",
  "gene_symbol": "PLAA"
}